{
  "gene_name": "Complement C1q tumor necrosis factor-related protein 6",
  "term_label": "extracellular space",
  "gene_symbol": "C1QTNF6",
  "gene": "UniProtKB:Q9BXI9",
  "term_id": "GO:0005615"
}